megagametogenesis [GO:0009561] (BP) Also known as: embryo sac development from the megaspore, megagametophyte nucleus division Definition: The process whose specific outcome is the progression of the embryo sac over time, from its formation as the megaspore to the mature structure. The process begins when three of the four haploid megaspores disintegrate, and the fourth undergoes mitosis giving rise to a binucleate syncytial embryo sac. The two haploid nuclei migrate to the opposite poles of the embryo sac and then undergo two rounds of mitosis generating four haploid nuclei at each pole. One nucleus from each set of four migrates to the center of the cell. Cellularization occurs, resulting in an eight-nucleate seven-celled structure. This structure contains two synergid cells and an egg cell at the micropylar end, and three antipodal cells at the other end. A binucleate endosperm mother cell is formed at the center. Sources: GOC:jl, GOC:mtg_plant Relationships: is a type of GO:0032501; is part of embryo sac development [GO:0009553]